{
  "term_label": "Unknown cellular component",
  "gene": "UniProtKB:A0A1B0GTQ1",
  "gene_symbol": "A0A1B0GTQ1",
  "gene_name": "Uncharacterized protein",
  "term_id": "UNKNOWN:0003"
}